cell wall (1->3)-beta-D-glucan biosynthetic process [GO:0034411] (BP) Definition: The chemical reactions and pathways resulting in the formation of (1->3)-beta-D-glucans, compounds composed of glucose residues linked by (1->3)-beta-D-glucosidic bonds, found in the walls of cells. Regulation: regulated by regulation of cell wall (1->3)-beta-D-glucan biosynthetic process [GO:0090334] Also known as: cell wall 1,3-beta-D-glucan biosynthetic process, cell wall 1,3-beta-glucan biosynthetic process, cell wall 1,3-beta-glucan anabolism, cell wall 1,3-beta-glucan biosynthesis, cell wall 1,3-beta-glucan formation, cell wall 1,3-beta-glucan synthesis, cell wall beta-1,3-glucan anabolism, cell wall beta-1,3-glucan biosynthesis, cell wall beta-1,3-glucan biosynthetic process, cell wall beta-1,3-glucan formation, cell wall beta-1,3-glucan synthesis Sources: GOC:mah Relationships: is a type of (1->3)-beta-D-glucan biosynthetic process [GO:0006075]; is a type of cell wall (1->3)-beta-D-glucan metabolic process [GO:0034407]; is_a cell wall beta-glucan biosynthetic process [GO:0034410] Subtypes: fungal-type cell wall (1->3)-beta-D-glucan biosynthetic process [GO:0071970]